{
  "gene_name": "Neuroglobin",
  "term_label": "response to hypoxia",
  "gene_symbol": "NGB",
  "term_id": "GO:0001666",
  "gene": "UniProtKB:Q9NPG2"
}